{
  "gene_symbol": "C11orf54",
  "term_label": "Unknown biological process",
  "gene": "UniProtKB:Q9H0W9",
  "gene_name": "Ester hydrolase C11orf54",
  "term_id": "UNKNOWN:0002"
}